regulation of transcription open complex formation at RNA polymerase II promoter [GO:0001177] (biological process) Also known as: regulation of transcriptional open complex formation at RNA polymerase II promoter Sources: GOC:txnOH Relationships: is a type of regulation of cellular component organization [GO:0051128]; regulates transcription open complex formation at RNA polymerase II promoter [GO:0001113] Definition: Any process that modulates the rate, frequency or extent of a process involved the melting of the DNA hybrid of the core promoter region within the transcriptional closed complex of an RNA polymerase II preinitiation complex (PIC) to produce an open complex where the DNA duplex around the transcription initiation site is unwound to form the transcription bubble.